{
  "gene_symbol": "ENAM",
  "term_id": "GO:0031012",
  "gene_name": "Enamelin",
  "gene": "UniProtKB:Q9NRM1",
  "term_label": "extracellular matrix"
}